{
  "term_label": "DNA helicase activity",
  "gene_name": "Probable ATP-dependent DNA helicase HFM1",
  "term_id": "GO:0003678",
  "gene": "UniProtKB:A2PYH4",
  "gene_symbol": "HFM1"
}